protein-phosphoribosyl dephospho-coenzyme A linkage [GO:0018247] (biological process) Relationships: is a type of peptidyl-serine modification [GO:0018209]; is a type of protein-coenzyme A linkage [GO:0018246] Definition: The linkage of phosphoribosyl dephospho-coenzyme A to protein via peptidyl-serine, to form O-(phosphoribosyl dephospho-coenzyme A)-L-serine; it is uncertain whether the phosphoribosyl glycosidic attachment to the dephospho-coenzyme A is alpha or beta, and through the 2' or the 3' position. Sources: RESID:AA0167